{
  "gene_name": "Dynein regulatory complex protein 11",
  "term_id": "GO:0005634",
  "gene": "UniProtKB:Q86XH1",
  "term_label": "nucleus",
  "gene_symbol": "IQCA1"
}